{
  "gene_name": "P2Y purinoceptor 13",
  "gene": "UniProtKB:Q9BPV8",
  "term_label": "G protein-coupled purinergic nucleotide receptor activity",
  "term_id": "GO:0045028",
  "gene_symbol": "P2RY13"
}